mitral valve development [GO:0003174] (biological process) Sources: GOC:mtg_heart Relationships: is a type of GO:0003171 Definition: The progression of the mitral valve over time, from its formation to the mature structure.